{
  "gene": "UniProtKB:P19827",
  "term_id": "UNKNOWN:0001",
  "gene_name": "Inter-alpha-trypsin inhibitor heavy chain H1",
  "gene_symbol": "ITIH1",
  "term_label": "Unknown molecular function"
}